{
  "gene_name": "ADP-ribosylation factor-like protein 1",
  "term_id": "GO:0006886",
  "gene": "UniProtKB:P40616",
  "term_label": "intracellular protein transport",
  "gene_symbol": "ARL1"
}